{
  "gene_symbol": "REXO1",
  "gene": "UniProtKB:Q8N1G1",
  "term_id": "GO:0004527",
  "term_label": "exonuclease activity",
  "gene_name": "RNA exonuclease 1 homolog"
}